{
  "gene_name": "Low-density lipoprotein receptor-related protein 12",
  "term_label": "Unknown biological process",
  "gene": "UniProtKB:Q9Y561",
  "gene_symbol": "LRP12",
  "term_id": "UNKNOWN:0002"
}